{
  "gene": "UniProtKB:Q6STE5",
  "gene_name": "SWI_SNF-related matrix-associated actin-dependent regulator of chromatin subfamily D member 3",
  "gene_symbol": "SMARCD3",
  "term_id": "GO:0003712",
  "term_label": "transcription coregulator activity"
}